{
  "term_label": "plasma membrane",
  "gene": "UniProtKB:Q9H210",
  "term_id": "GO:0005886",
  "gene_name": "Olfactory receptor 2D2",
  "gene_symbol": "OR2D2"
}